postsynapse of neuromuscular junction [GO:0098975] (cellular component) Definition: The postsynapse of a neuromuscular junction. In vertebrate muscles this includes the motor end-plate, consisting of postjunctional folds of the sarcolemma. Relationships: is a type of GO:0098794; BFO_0000050 neuromuscular junction [GO:0031594] Sources: GOC:dos, Wikipedia:Neuromuscular_junction&oldid=723623502